{
  "gene_name": "Putative beta-defensin 108A",
  "term_id": "UNKNOWN:0002",
  "gene_symbol": "DEFB108C",
  "term_label": "Unknown biological process",
  "gene": "UniProtKB:A8MXU0"
}